{
  "gene_symbol": "CST5",
  "gene_name": "Cystatin-D",
  "term_label": "extracellular space",
  "gene": "UniProtKB:P28325",
  "term_id": "GO:0005615"
}